erythromycin biosynthetic process [GO:1901115] (biological process) Definition: The chemical reactions and pathways resulting in the formation of erythromycin. Also known as: erythromycin anabolism, erythromycin biosynthesis, erythromycin formation, erythromycin synthesis Relationships: is_a GO:0033068 Sources: GOC:TermGenie, GOC:yaf, UniPathway:UPA00240